retromer complex binding [GO:1905394] (molecular function) Relationships: is a type of protein-containing complex binding [GO:0044877] Definition: Binding to a retromer complex. References: PMID:27385586 Sources: GOC:PARL, GOC:TermGenie, GOC:bc